tRNA dimethylallyltransferase activity [GO:0052381] (molecular function) Definition: Catalysis of the reaction: adenosine(37) in tRNA + dimethylallyl diphosphate = N(6)-dimethylallyladenosine(37) in tRNA + diphosphate. Sources: EC:2.5.1.75, RHEA:26482 Also known as: tRNA prenyltransferase activity, dimethylallyl-diphosphate:tRNA dimethylallyltransferase activity, tRNA N6-adenosine-37 dimethylallyltransferase activity, tRNA isopentenyltransferase activity Note: Note that this activity was formerly know in GO and EC as 'tRNA isopentenyltransferase' (GO:0004811), but it is now known that dimethylallyl diphosphate, rather than isopentenyl diphosphate, is the substrate. Relationships: is_a transferase activity, transferring alkyl or aryl (other than methyl) groups [GO:0016765]; is a type of catalytic activity, acting on a tRNA [GO:0140101]